{
  "gene_name": "Tyrosine-protein phosphatase non-receptor type 7",
  "gene": "UniProtKB:P35236",
  "term_label": "protein tyrosine phosphatase activity",
  "term_id": "GO:0004725",
  "gene_symbol": "PTPN7"
}